{
  "gene_symbol": "HCRT",
  "gene_name": "Hypocretin neuropeptide precursor",
  "gene": "UniProtKB:O43612",
  "term_id": "GO:0042594",
  "term_label": "response to starvation"
}